{
  "gene_symbol": "PRSS22",
  "gene_name": "Brain-specific serine protease 4",
  "term_label": "Unknown cellular component",
  "gene": "UniProtKB:Q9GZN4",
  "term_id": "UNKNOWN:0003"
}